protein localization to T cell secretory granule [GO:0033374] (biological process) Definition: A process in which a protein is transported to, or maintained in, a location within a secretory granule in a T cell. Also known as: protein localisation in T cell secretory granule, protein localization in T cell secretory granule, protein localization in T lymphocyte secretory granule, protein localization in T-cell secretory granule, protein localization in T-lymphocyte secretory granule Relationships: is a type of protein localization to secretory granule [GO:0033366]; is part of T cell secretory granule organization [GO:0033371] Subtypes: protease localization to T cell secretory granule [GO:0033375] Sources: GOC:mah